penta-snRNP complex [GO:0071003] (cellular component) Relationships: is a type of spliceosomal snRNP complex [GO:0097525]; has part U5 snRNP [GO:0005682]; has part U1 snRNP [GO:0005685]; has part U2 snRNP [GO:0005686]; has part U4/U6 snRNP [GO:0071001] References: PMID:11804584, PMID:12724403 Sources: GOC:krc, GOC:mah Also known as: penta-RNP complex Definition: A ribonucleoprotein complex that is formed by the association of the U1, U2, U4/U6 and U5 small nuclear ribonucleoproteins.